chlorogenate-glucarate O-hydroxycinnamoyltransferase activity [GO:0047204] (MF) Definition: Catalysis of the reaction: D-glucarate + chlorogenate = (-)-quinate + 2-O-caffeoylglucarate. Also known as: chlorogenate:glucarate O-(hydroxycinnamoyl)transferase activity, chlorogenate:glucarate caffeoyltransferase activity, chlorogenic acid:glucaric acid O-caffeoyltransferase activity Sources: EC:2.3.1.98, RHEA:23204 Relationships: is a type of O-hydroxycinnamoyltransferase activity [GO:0050737]